{
  "gene_symbol": "EXOSC10",
  "gene_name": "Exosome component 10",
  "gene": "UniProtKB:Q01780",
  "term_label": "TRAMP-dependent tRNA surveillance pathway",
  "term_id": "GO:0071038"
}